{
  "term_id": "GO:0098609",
  "gene": "UniProtKB:Q13349",
  "gene_name": "Integrin alpha-D",
  "gene_symbol": "ITGAD",
  "term_label": "cell-cell adhesion"
}